D-ribose transmembrane transporter activity [GO:0015591] (molecular function) Sources: GOC:mtg_transport, ISBN:0198506732, ISBN:0815340729 Relationships: is a type of GO:0015146; is part of D-ribose transmembrane transport [GO:0015752] Subtypes: ABC-type D-ribose transporter activity [GO:0015611] Definition: Enables the transfer of D-ribose from one side of a membrane to the other. As beta-D-ribofuranose, D-ribose forms the glycose group of all ribonucleosides, ribonucleotides and ribonucleic acids, and also of ribose phosphates, various glycosides, some coenzymes and some forms of vitamin B12.